regulation of cell proliferation in dorsal spinal cord [GO:0021921] (biological process) Definition: The process that modulates the frequency, rate or extent of cell proliferation in the dorsal spinal cord. Subtypes: negative regulation of cell proliferation in dorsal spinal cord [GO:1902832], positive regulation of cell proliferation in dorsal spinal cord [GO:1902833] Relationships: is a type of regulation of neural precursor cell proliferation [GO:2000177]; is part of dorsal spinal cord development [GO:0021516]; regulates cell proliferation in dorsal spinal cord [GO:0010456] Sources: GOC:cls, GOC:dgh, GOC:dph, GOC:jid, GO_REF:0000021